{
  "gene_symbol": "PRSS58",
  "gene": "UniProtKB:Q8IYP2",
  "gene_name": "Serine protease 58",
  "term_label": "extracellular space",
  "term_id": "GO:0005615"
}